{
  "gene_name": "Kinesin-like protein KIF24",
  "term_label": "microtubule motor activity",
  "gene": "UniProtKB:Q5T7B8",
  "term_id": "GO:0003777",
  "gene_symbol": "KIF24"
}